{
  "gene_symbol": "TP73",
  "term_label": "DNA-binding transcription factor activity, RNA polymerase II-specific",
  "term_id": "GO:0000981",
  "gene": "UniProtKB:O15350",
  "gene_name": "Tumor protein p73"
}